{
  "term_id": "UNKNOWN:0001",
  "gene": "UniProtKB:Q8WUQ7",
  "gene_symbol": "CACTIN",
  "gene_name": "Splicing factor Cactin",
  "term_label": "Unknown molecular function"
}